regulation of Golgi inheritance [GO:0090170] (BP) Definition: Any process that modulates the rate, frequency or extent of Golgi inheritance. Golgi inheritance is the partitioning of Golgi apparatus between daughter cells at cell division. Relationships: is a type of regulation of Golgi organization [GO:1903358]; regulates Golgi inheritance [GO:0048313] Sources: GOC:ascb_2009, GOC:dph, GOC:tb